{
  "term_label": "Unknown biological process",
  "gene_symbol": "OBP2A",
  "term_id": "UNKNOWN:0002",
  "gene_name": "Odorant-binding protein 2a",
  "gene": "UniProtKB:Q9NY56"
}